mesonephric duct formation [GO:0072181] (biological process) Relationships: is a type of GO:0072172; is a type of GO:0072179; is a type of mesonephric duct morphogenesis [GO:0072180] Sources: GOC:mtg_kidney_jan10 Definition: The developmental process pertaining to the initial formation of a mesonephric duct. A mesonephric duct is a tube that drains the mesonephros. Also known as: Wolffian duct formation